{
  "gene": "UniProtKB:P78382",
  "term_label": "CMP-N-acetylneuraminate transmembrane transport",
  "term_id": "GO:0015782",
  "gene_symbol": "SLC35A1",
  "gene_name": "CMP-sialic acid transporter"
}